{
  "gene_name": "Caveolin-3",
  "gene_symbol": "CAV3",
  "term_label": "cell differentiation",
  "term_id": "GO:0030154",
  "gene": "UniProtKB:P56539"
}